{
  "gene": "UniProtKB:Q9C009",
  "gene_symbol": "FOXQ1",
  "term_label": "regulation of transcription by RNA polymerase II",
  "gene_name": "Forkhead box protein Q1",
  "term_id": "GO:0006357"
}